{
  "term_label": "extracellular space",
  "term_id": "GO:0005615",
  "gene_name": "Podocan-like protein 1",
  "gene": "UniProtKB:Q6PEZ8",
  "gene_symbol": "PODNL1"
}